{
  "term_id": "GO:0016491",
  "gene": "UniProtKB:P49447",
  "term_label": "oxidoreductase activity",
  "gene_symbol": "CYB561",
  "gene_name": "Transmembrane ascorbate-dependent reductase CYB561"
}